cellular response to acrylamide [GO:1903938] (biological process) Relationships: is a type of cellular response to nitrogen compound [GO:1901699]; is a type of cellular response to oxygen-containing compound [GO:1901701]; is a type of GO:1903937 References: PMID:16292499 Sources: GOC:TermGenie, GO_REF:0000071 Definition: Any process that results in a change in state or activity of a cell (in terms of movement, secretion, enzyme production, gene expression, etc.) as a result of an acrylamide stimulus.